{
  "gene": "UniProtKB:Q16378",
  "term_label": "Unknown molecular function",
  "gene_name": "Proline-rich protein 4",
  "term_id": "UNKNOWN:0001",
  "gene_symbol": "PRR4"
}